{
  "term_id": "UNKNOWN:0002",
  "gene_symbol": "CHAD",
  "gene": "UniProtKB:O15335",
  "gene_name": "Chondroadherin",
  "term_label": "Unknown biological process"
}